vascular associated smooth muscle cell development [GO:0097084] (biological process) Sources: GOC:BHF Relationships: is a type of muscle cell development [GO:0055001]; is part of vascular associated smooth muscle cell differentiation [GO:0035886] Also known as: vascular smooth muscle cell development Definition: The process aimed at the progression of a vascular smooth muscle cell over time, from initial commitment of the cell to a specific fate, to the fully functional differentiated cell. A vascular smooth muscle cell is a non-striated, elongated, spindle-shaped cell found lining the blood vessels. Subtypes: cardiac vascular smooth muscle cell development [GO:0060948]